{
  "gene_name": "A-kinase anchor protein 13",
  "term_id": "GO:0015629",
  "gene_symbol": "AKAP13",
  "term_label": "actin cytoskeleton",
  "gene": "UniProtKB:Q12802"
}